{
  "gene_name": "Solute carrier family 15 member 3",
  "term_label": "dipeptide import across plasma membrane",
  "gene": "UniProtKB:Q8IY34",
  "gene_symbol": "SLC15A3",
  "term_id": "GO:0140206"
}